violaceol II metabolic process [GO:1900591] (biological process) Also known as: violaceol II metabolism Definition: The chemical reactions and pathways involving violaceol II. Subtypes: violaceol II catabolic process [GO:1900592], GO:1900593 Sources: GOC:TermGenie, GOC:di Relationships: is a type of catechol-containing compound metabolic process [GO:0009712]; is a type of secondary metabolic process [GO:0019748]